{
  "gene_symbol": "PCLO",
  "gene_name": "Protein piccolo",
  "term_id": "GO:0048788",
  "gene": "UniProtKB:Q9Y6V0",
  "term_label": "cytoskeleton of presynaptic active zone"
}